type 2 neuromedin U receptor binding [GO:0031840] (molecular function) Definition: Binding to a type 2 neuromedin U receptor. Sources: GOC:mah, GOC:nln Also known as: type 2 neuromedin U receptor ligand Relationships: is a type of neuromedin U receptor binding [GO:0042922]